positive regulation of proteasomal protein catabolic process [GO:1901800] (biological process) References: PMID:21669198 Sources: GOC:BHF, GOC:TermGenie, GOC:rl Relationships: is a type of positive regulation of protein catabolic process [GO:0045732]; is a type of regulation of proteasomal protein catabolic process [GO:0061136]; is_a GO:1903052; positively regulates proteasomal protein catabolic process [GO:0010498] Also known as: activation of proteasome-mediated protein catabolic process, activation of proteasome-mediated protein catabolism, positive regulation of proteasome-mediated protein catabolic process, positive regulation of proteasome-mediated protein catabolism, up regulation of proteasomal protein catabolic process, up regulation of proteasome-mediated protein catabolic process, up regulation of proteasome-mediated protein catabolism, up-regulation of proteasomal protein catabolic process, up-regulation of proteasome-mediated protein catabolic process, up-regulation of proteasome-mediated protein catabolism, upregulation of proteasomal protein catabolic process, upregulation of proteasome-mediated protein catabolic process, upregulation of proteasome-mediated protein catabolism, activation of proteasomal protein catabolic process Definition: Any process that activates or increases the frequency, rate or extent of proteasomal protein catabolic process. Subtypes: GO:0032436, positive regulation of ERAD pathway [GO:1904294]